regulation of COPII vesicle coating [GO:0003400] (biological process) Relationships: is a type of regulation of organelle organization [GO:0033043]; is a type of regulation of protein-containing complex assembly [GO:0043254]; regulates COPII vesicle coating [GO:0048208] Sources: GOC:ascb_2009, GOC:dph, GOC:jp, GOC:tb Definition: Any process that modulates the rate, frequency, or extent of the addition of COPII proteins and adaptor proteins to ER membranes during the formation of transport vesicles, forming a vesicle coat.